dipeptide import across plasma membrane [GO:0140206] (biological process) Definition: The directed movement of a dipeptide from outside of a cell, across the plasma membrane and into the cytosol. Relationships: is a type of dipeptide transmembrane transport [GO:0035442]; is a type of GO:0140205 References: PMID:22226946